{
  "term_label": "PRC1 complex",
  "gene": "UniProtKB:Q86SE9",
  "gene_symbol": "PCGF5",
  "gene_name": "Polycomb group RING finger protein 5",
  "term_id": "GO:0035102"
}